endothelial cell chemotaxis [GO:0035767] (biological process) Definition: The directed movement of an endothelial cell guided by a specific chemical concentration gradient. Movement may be towards a higher concentration (positive chemotaxis) or towards a lower concentration (negative chemotaxis). Regulation: regulated by regulation of endothelial cell chemotaxis [GO:2001026]; RO_0002212 by negative regulation of endothelial cell chemotaxis [GO:2001027]; positively regulated by positive regulation of endothelial cell chemotaxis [GO:2001028] Subtypes: GO:0035768 Sources: CL:0000115, GOC:BHF Relationships: is_a endothelial cell migration [GO:0043542]; is a type of cell chemotaxis [GO:0060326]